cullin family protein binding [GO:0097602] (molecular function) Relationships: is a type of GO:0005515 References: PMID:18698375 Sources: GOC:ha, InterPro:IPR016158 Also known as: cullin binding Definition: Binding to a member of the cullin family, hydrophobic proteins that act as scaffolds for ubiquitin ligases (E3).